{
  "gene_symbol": "SH2B3",
  "term_id": "GO:0005068",
  "term_label": "transmembrane receptor protein tyrosine kinase adaptor activity",
  "gene": "UniProtKB:Q9UQQ2",
  "gene_name": "SH2B adapter protein 3"
}